{
  "gene": "UniProtKB:P11216",
  "gene_name": "Glycogen phosphorylase, brain form",
  "gene_symbol": "PYGB",
  "term_id": "GO:0008184",
  "term_label": "glycogen phosphorylase activity"
}